xenobiotic transport [GO:0042908] (biological process) Also known as: drug transport Definition: The directed movement of a xenobiotic into, out of or within a cell, or between cells, by means of some agent such as a transporter or pore. A xenobiotic is a compound foreign to the organism exposed to it. It may be synthesized by another organism (like ampicilin) or it can be a synthetic chemical. Relationships: is a type of transport [GO:0006810] Sources: GOC:go_curators, GOC:krc Subtypes: xenobiotic transmembrane transport [GO:0006855], xenobiotic export from cell [GO:0046618], xenobiotic transport across blood-nerve barrier [GO:0061772], xenobiotic detoxification by transmembrane export across the cell outer membrane [GO:0140330], xenobiotic transport across blood-brain barrier [GO:1990962]